{
  "gene": "UniProtKB:Q16627",
  "gene_name": "C-C motif chemokine 14",
  "term_id": "GO:0048020",
  "gene_symbol": "CCL14",
  "term_label": "CCR chemokine receptor binding"
}